{
  "term_id": "UNKNOWN:0001",
  "gene": "UniProtKB:Q8TDP1",
  "gene_symbol": "RNASEH2C",
  "gene_name": "Ribonuclease H2 subunit C",
  "term_label": "Unknown molecular function"
}